{
  "gene_symbol": "ZNF333",
  "term_id": "GO:0000981",
  "gene": "UniProtKB:Q96JL9",
  "gene_name": "Zinc finger protein 333",
  "term_label": "DNA-binding transcription factor activity, RNA polymerase II-specific"
}